response to salt [GO:1902074] (biological process) Subtypes: GO:1902075, GO:1903935, response to sodium phosphate [GO:1904383] References: PMID:16666921 Sources: GOC:TermGenie, GOC:mls Also known as: response to salinity Relationships: is_a response to chemical [GO:0042221] Definition: Any process that results in a change in state or activity of a cell or an organism (in terms of movement, secretion, enzyme production, gene expression, etc.) as a result of a salt stimulus.